ribitol catabolic process to D-xylulose 5-phosphate [GO:0019488] (biological process) Definition: The chemical reactions and pathways resulting in the breakdown of ribitol to form D-xylulose 5-phosphate. Ribitol is initially converted to D-ribulose, which is phosphorylated to form D-ribulose 5-phosphate, which is then converted into D-xylulose 5-phosphate. Sources: MetaCyc:RIBITOLUTIL-PWY Also known as: ribitol breakdown to xylulose 5-phosphate, ribitol degradation to xylulose 5-phosphate, ribitol utilization Relationships: is a type of GO:0046363; is_a D-xylulose 5-phosphate metabolic process [GO:0051167]